{
  "gene_symbol": "MARK4",
  "gene_name": "MAP_microtubule affinity-regulating kinase 4",
  "term_label": "tau-protein kinase activity",
  "term_id": "GO:0050321",
  "gene": "UniProtKB:Q96L34"
}